{
  "gene": "UniProtKB:Q3SXM0",
  "term_id": "UNKNOWN:0001",
  "gene_name": "DDB1- and CUL4-associated factor 4-like protein 1",
  "gene_symbol": "DCAF4L1",
  "term_label": "Unknown molecular function"
}